cAMP-dependent protein kinase complex [GO:0005952] (cellular component) Definition: An enzyme complex, composed of regulatory and catalytic subunits, that catalyzes protein phosphorylation. Inactive forms of the enzyme have two regulatory chains and two catalytic chains; activation by cAMP produces two active catalytic monomers and a regulatory dimer. References: PMID:18178622 Also known as: 3',5' cAMP-dependent protein kinase complex, 3',5'-cAMP-dependent protein kinase complex, adenosine 3',5'-cyclophosphate-dependent protein kinase complex, cyclic AMP-dependent protein kinase complex, PKA Relationships: is a type of intracellular protein-containing complex [GO:0140535]; is a type of serine/threonine protein kinase complex [GO:1902554]